negative regulation of establishment of endothelial barrier [GO:1903141] (biological process) References: PMID:24851274 Sources: GOC:TermGenie, GOC:als, GO_REF:0000058 Relationships: is a type of negative regulation of endothelial cell development [GO:1901551]; is a type of regulation of establishment of endothelial barrier [GO:1903140]; negatively regulates GO:0061028 Definition: Any process that stops, prevents or reduces the frequency, rate or extent of establishment of endothelial barrier. Also known as: down regulation of establishment of endothelial barrier, down-regulation of establishment of endothelial barrier, downregulation of establishment of endothelial barrier, inhibition of establishment of endothelial barrier